regulation of vitamin metabolic process [GO:0030656] (biological process) Also known as: regulation of vitamin metabolism Sources: GOC:mah Relationships: is a type of regulation of small molecule metabolic process [GO:0062012]; regulates vitamin metabolic process [GO:0006766] Definition: Any process that modulates the frequency, rate or extent of the chemical reactions and pathways involving a vitamin, one of a number of unrelated organic substances that occur in many foods in small amounts and that are necessary in trace amounts for the normal metabolic functioning of the body. Subtypes: positive regulation of vitamin metabolic process [GO:0046136], negative regulation of vitamin metabolic process [GO:0046137], regulation of vitamin D biosynthetic process [GO:0060556], regulation of thiamine diphosphate biosynthetic process [GO:0070616], regulation of thiamine biosynthetic process [GO:0070623], GO:1900052, regulation of vitamin E biosynthetic process [GO:1904965], GO:2000082